{
  "gene_symbol": "PDLIM5",
  "term_label": "muscle alpha-actinin binding",
  "term_id": "GO:0051371",
  "gene": "UniProtKB:Q96HC4",
  "gene_name": "PDZ and LIM domain protein 5"
}